{
  "term_label": "cytosol",
  "gene_symbol": "ACLY",
  "term_id": "GO:0005829",
  "gene": "UniProtKB:P53396",
  "gene_name": "ATP-citrate synthase"
}